{
  "term_label": "Golgi membrane",
  "term_id": "GO:0000139",
  "gene_symbol": "UNC50",
  "gene_name": "Protein unc-50 homolog",
  "gene": "UniProtKB:Q53HI1"
}